regulation of epidermal cell division [GO:0010482] (BP) Definition: Any process that modulates the frequency, rate or extent of the physical partitioning and separation of an epidermal cell into daughter cells. An epidermal cell is any of the cells that make up the epidermis. References: PMID:17450124 Also known as: regulation of hypodermal cell division Relationships: is_a regulation of cell division [GO:0051302]; regulates GO:0010481